{
  "gene_symbol": "GORASP2",
  "gene": "UniProtKB:Q9H8Y8",
  "term_id": "GO:0005794",
  "gene_name": "Golgi reassembly-stacking protein 2",
  "term_label": "Golgi apparatus"
}